{
  "gene_symbol": "BMS1",
  "gene": "UniProtKB:Q14692",
  "term_label": "RNA binding",
  "term_id": "GO:0003723",
  "gene_name": "Ribosome biogenesis protein BMS1 homolog"
}